{
  "gene_symbol": "GSDMD",
  "term_label": "NLRP3 inflammasome complex",
  "term_id": "GO:0072559",
  "gene": "UniProtKB:P57764",
  "gene_name": "Gasdermin-D"
}